{
  "term_label": "adenylate cyclase-activating G protein-coupled receptor signaling pathway",
  "term_id": "GO:0007189",
  "gene_name": "Growth hormone-releasing hormone receptor",
  "gene": "UniProtKB:Q02643",
  "gene_symbol": "GHRHR"
}